{
  "gene_name": "PRAME family member 18",
  "term_label": "ubiquitin-like ligase-substrate adaptor activity",
  "gene": "UniProtKB:Q5VWM3",
  "term_id": "GO:1990756",
  "gene_symbol": "PRAMEF18"
}